{
  "gene_name": "Roundabout homolog 4",
  "term_label": "plasma membrane",
  "term_id": "GO:0005886",
  "gene": "UniProtKB:Q8WZ75",
  "gene_symbol": "ROBO4"
}